{
  "gene_name": "Early lymphoid activation gene protein",
  "gene": "UniProtKB:Q14236",
  "term_id": "UNKNOWN:0003",
  "gene_symbol": "DIAPH2-AS1",
  "term_label": "Unknown cellular component"
}